acetylglutamate kinase regulator activity [GO:0010307] (molecular function) Relationships: is a type of kinase regulator activity [GO:0019207]; regulates acetylglutamate kinase activity [GO:0003991] Definition: Binds to and modulates the activity of acetylglutamate kinase. References: PMID:16377628